lipooligosaccharide binding [GO:1990458] (molecular function) Definition: Binding to lipooligosaccharide. Lipooligosaccharides (LOSs) are the major glycolipids expressed on mucosal Gram-negative bacteria. Note: ChEBI distinguishes an oligosaccharide from a polysaccharide as the latter being anything of length 10 or greater. Also known as: LOS binding, endotoxin binding Relationships: is_a carbohydrate derivative binding [GO:0097367] References: PMID:8894399 Sources: GOC:hjd